polyspecific organic cation:proton antiporter activity [GO:0140968] (molecular function) Relationships: is_a proton transmembrane transporter activity [GO:0015078]; is a type of GO:0015297 Also known as: proton:polyspecific organic cation antiporter activity Definition: Enables the transfer of various organic cations in exchange for a proton, according to the reaction: H+(out) + organic cation(in) = H+(in) + organic cation(out). The transported substrates are usually toxic molecules, drugs and xenobiotics. References: PMID:17047166, PMID:17509534